{
  "gene_symbol": "GTF2I",
  "gene_name": "General transcription factor II-I",
  "gene": "UniProtKB:P78347",
  "term_id": "GO:0003700",
  "term_label": "DNA-binding transcription factor activity"
}